{
  "term_id": "GO:0006809",
  "term_label": "nitric oxide biosynthetic process",
  "gene": "UniProtKB:P16435",
  "gene_name": "NADPH--cytochrome P450 reductase",
  "gene_symbol": "POR"
}